{
  "gene_symbol": "MRE11",
  "term_id": "GO:0097552",
  "gene": "UniProtKB:P49959",
  "term_label": "mitochondrial double-strand break repair via homologous recombination",
  "gene_name": "Double-strand break repair protein MRE11"
}